{
  "gene": "UniProtKB:O95292",
  "gene_name": "Vesicle-associated membrane protein-associated protein B_C",
  "term_label": "endoplasmic reticulum membrane",
  "gene_symbol": "VAPB",
  "term_id": "GO:0005789"
}